{
  "gene": "UniProtKB:Q86XW9",
  "term_id": "UNKNOWN:0001",
  "term_label": "Unknown molecular function",
  "gene_name": "Thioredoxin domain-containing protein 6",
  "gene_symbol": "NME9"
}